negative regulation of lens fiber cell differentiation [GO:1902747] (biological process) Also known as: down regulation of lens fiber cell differentiation, down regulation of lens fibre cell differentiation, down-regulation of lens fiber cell differentiation, down-regulation of lens fibre cell differentiation, downregulation of lens fiber cell differentiation, downregulation of lens fibre cell differentiation, negative regulation of lens fibre cell differentiation, inhibition of lens fiber cell differentiation, inhibition of lens fibre cell differentiation References: PMID:17592637 Sources: GOC:TermGenie, GOC:mr, GO_REF:0000058 Relationships: is a type of negative regulation of epithelial cell differentiation [GO:0030857]; is_a negative regulation of multicellular organismal process [GO:0051241]; is a type of regulation of lens fiber cell differentiation [GO:1902746]; negatively regulates lens fiber cell differentiation [GO:0070306] Definition: Any process that stops, prevents or reduces the frequency, rate or extent of lens fiber cell differentiation.